{
  "term_label": "ADP binding",
  "gene_name": "ATP synthase subunit alpha, mitochondrial",
  "gene_symbol": "ATP5F1A",
  "term_id": "GO:0043531",
  "gene": "UniProtKB:P25705"
}